ureidoglycine aminohydrolase activity [GO:0071522] (molecular function) Definition: Catalysis of the reaction: ureidoglycine + H2O = S-ureidoglycolate + NH3. References: PMID:19935661, PMID:20038185 Sources: MetaCyc:URUR-RXN Relationships: is a type of hydrolase activity, acting on carbon-nitrogen (but not peptide) bonds, in linear amidines [GO:0016813]